response to putrescine [GO:1904585] (BP) Definition: Any process that results in a change in state or activity of a cell or an organism (in terms of movement, secretion, enzyme production, gene expression, etc.) as a result of a putrescine stimulus. Subtypes: GO:1904586 References: PMID:20805360 Sources: GOC:TermGenie, GO_REF:0000071 Also known as: response to 1,4-Butanediamine, response to 1,4-Diaminobutane, response to tetramethylenediamine Relationships: is a type of response to nitrogen compound [GO:1901698]